{
  "gene_name": "STE20-related kinase adapter protein beta",
  "gene": "UniProtKB:Q9C0K7",
  "term_label": "protein serine/threonine kinase activator activity",
  "term_id": "GO:0043539",
  "gene_symbol": "STRADB"
}